{
  "gene_name": "Lysine-specific demethylase 6A",
  "term_label": "MLL3/4 complex",
  "gene": "UniProtKB:O15550",
  "gene_symbol": "KDM6A",
  "term_id": "GO:0044666"
}